leukotriene-B4 20-monooxygenase activity [GO:0050051] (molecular function) Also known as: LTB(4) 20-hydroxylase activity, LTB(4) omega-hydroxylase activity, LTB4 20-hydroxylase activity, LTB4 omega-hydroxylase activity, leukotriene-B4 20-hydroxylase activity, leukotriene-B4 omega-hydroxylase activity References: PMID:11461919, PMID:15364545, PMID:8486631, PMID:9675028 Sources: RHEA:22176 Relationships: is a type of oxidoreductase activity, acting on paired donors, with incorporation or reduction of molecular oxygen, reduced flavin or flavoprotein as one donor, and incorporation of one atom of oxygen [GO:0016712]; is part of leukotriene B4 catabolic process [GO:0036101] Definition: Catalysis of the reaction: leukotriene B4 + O2 + reduced [NADPH-hemoprotein reductase] = 20-hydroxy-leukotriene B4 + H+ + H2O + oxidized [NADPH-hemoprotein reductase].